{
  "gene_symbol": "STRN",
  "gene": "UniProtKB:O43815",
  "term_id": "GO:0098794",
  "gene_name": "Striatin",
  "term_label": "postsynapse"
}